protein transport into membrane raft [GO:0032596] (biological process) Also known as: protein translocation into membrane raft, protein transport into lipid raft, receptor translocation into membrane raft, receptor transport into membrane raft Definition: The directed movement of a protein into a membrane raft. Membrane rafts are small (10-200 nm), heterogeneous, highly dynamic, sterol- and sphingolipid-enriched membrane domains that compartmentalize cellular processes. Sources: GOC:mah Relationships: is a type of protein transport within lipid bilayer [GO:0032594]; is a type of establishment of protein localization to membrane [GO:0090150]; is a type of protein localization to membrane raft [GO:1903044] Subtypes: B cell receptor transport into membrane raft [GO:0032597], protein transport into plasma membrane raft [GO:0044861]